trachea formation [GO:0060440] (biological process) Definition: The process pertaining to the initial formation of a trachea from unspecified parts. The process begins with the specific processes that contribute to the appearance of the discrete structure and ends when the trachea is recognizable. The trachea is the portion of the airway that attaches to the bronchi as it branches. Sources: GOC:dph Relationships: is a type of animal organ formation [GO:0048645]; is part of GO:0060439